{
  "gene_name": "Two pore channel protein 2",
  "term_id": "GO:0015280",
  "gene": "UniProtKB:Q8NHX9",
  "gene_symbol": "TPCN2",
  "term_label": "ligand-gated sodium channel activity"
}